{
  "term_id": "GO:0072676",
  "gene_symbol": "TBX21",
  "term_label": "lymphocyte migration",
  "gene": "UniProtKB:Q9UL17",
  "gene_name": "T-box transcription factor TBX21"
}